ethyl acetate biosynthetic process [GO:1902819] (biological process) Relationships: is a type of GO:0009058 References: PMID:16013377 Sources: GOC:TermGenie, GOC:mengo_curators, GO_REF:0000068 Definition: The chemical reactions and pathways resulting in the formation of ethyl acetate. Also known as: ethyl acetate anabolism, ethyl acetate biosynthesis, ethyl acetate formation, ethyl acetate synthesis, ethyl ethanoate biosynthetic process